{
  "gene_symbol": "CCR10",
  "term_label": "external side of plasma membrane",
  "term_id": "GO:0009897",
  "gene_name": "C-C chemokine receptor type 10",
  "gene": "UniProtKB:P46092"
}